intracellular chemical homeostasis [GO:0055082] (biological process) Definition: A homeostatic process involved in the maintenance of a steady state level of a chemical within a cell. Subtypes: intracellular glucose homeostasis [GO:0001678], intracellular monoatomic ion homeostasis [GO:0006873], intracellular water homeostasis [GO:0009992], intracellular polyamine homeostasis [GO:0010509], GO:0030642, intracellular phosphate ion homeostasis [GO:0030643], intracellular oxygen homeostasis [GO:0032364], intracellular nitric oxide homeostasis [GO:0033484], intracellular triglyceride homeostasis [GO:0035356], intracellular acyl-CoA homeostasis [GO:0042049], intracellular amino acid homeostasis [GO:0080144], intracellular sphingolipid homeostasis [GO:0090156], intracellular ammonium homeostasis [GO:0097275], GO:0140964, intracellular nucleotide homeostasis [GO:0140979], GO:0140980, intracellular nitrogen homeostasis [GO:0141067], intracellular borate homeostasis [GO:0160070], intracellular abscisic acid homeostasis [GO:1902266] Also known as: cellular chemical homeostasis Sources: GOC:isa_complete, GOC:jid Relationships: is a type of cellular homeostasis [GO:0019725]; is a type of chemical homeostasis [GO:0048878]